endothelial microparticle formation [GO:0072565] (biological process) References: PMID:16373184 Sources: GOC:BHF, GOC:mah Definition: The cellular component organization process in which microparticles bud off from an endothelial cell. Relationships: is a type of blood microparticle formation [GO:0072564] Also known as: endothelial microparticle generation, endothelial microparticle release Regulation: regulated by regulation of endothelial microparticle formation [GO:2000335]; negatively regulated by GO:2000336; positively regulated by GO:2000337